{
  "term_id": "GO:0003823",
  "gene_name": "Immunoglobulin heavy variable 3_OR16-8 (non-functional) (Fragment)",
  "gene": "UniProtKB:A0A075B7F1",
  "gene_symbol": "IGHV3OR16-8",
  "term_label": "antigen binding"
}